{
  "gene": "UniProtKB:Q8N7H1",
  "term_label": "Unknown cellular component",
  "gene_name": "Putative uncharacterized protein encoded by LINC01465",
  "term_id": "UNKNOWN:0003",
  "gene_symbol": "LINC01465"
}